{
  "gene_name": "Parafibromin",
  "term_label": "positive regulation of transcription elongation by RNA polymerase II",
  "gene_symbol": "CDC73",
  "term_id": "GO:0032968",
  "gene": "UniProtKB:Q6P1J9"
}